{
  "term_label": "regulation of fatty acid beta-oxidation",
  "gene_name": "Peroxisomal leader peptide-processing protease",
  "gene": "UniProtKB:Q2T9J0",
  "gene_symbol": "TYSND1",
  "term_id": "GO:0031998"
}